{
  "gene": "UniProtKB:Q9H8X3",
  "term_id": "UNKNOWN:0003",
  "term_label": "Unknown cellular component",
  "gene_name": "Putative uncharacterized protein LINC00574",
  "gene_symbol": "LINC00574"
}